{
  "gene": "UniProtKB:Q8NG78",
  "term_id": "UNKNOWN:0003",
  "gene_symbol": "OR8G5",
  "gene_name": "Olfactory receptor 8G5",
  "term_label": "Unknown cellular component"
}